{
  "gene": "UniProtKB:Q16610",
  "term_label": "Unknown molecular function",
  "gene_name": "Extracellular matrix protein 1",
  "gene_symbol": "ECM1",
  "term_id": "UNKNOWN:0001"
}